{
  "gene": "UniProtKB:Q6UXC1",
  "gene_name": "Apical endosomal glycoprotein",
  "gene_symbol": "MAMDC4",
  "term_id": "UNKNOWN:0001",
  "term_label": "Unknown molecular function"
}